{
  "gene_symbol": "FGF21",
  "gene": "UniProtKB:Q9NSA1",
  "term_id": "GO:0008284",
  "term_label": "positive regulation of cell population proliferation",
  "gene_name": "Fibroblast growth factor 21"
}